{
  "term_label": "Unknown biological process",
  "gene_name": "ATP synthase subunit ATP5MJ, mitochondrial",
  "term_id": "UNKNOWN:0002",
  "gene": "UniProtKB:P56378",
  "gene_symbol": "ATP5MJ"
}